{
  "gene_name": "Serine_threonine-protein phosphatase 2A 55 kDa regulatory subunit B beta isoform",
  "gene_symbol": "PPP2R2B",
  "term_label": "protein phosphatase type 2A complex",
  "term_id": "GO:0000159",
  "gene": "UniProtKB:Q00005"
}